{
  "term_label": "regulation of transcription by RNA polymerase II",
  "gene": "UniProtKB:P48742",
  "term_id": "GO:0006357",
  "gene_symbol": "LHX1",
  "gene_name": "LIM_homeobox protein Lhx1"
}